{
  "term_id": "GO:0045944",
  "gene": "UniProtKB:O43151",
  "term_label": "positive regulation of transcription by RNA polymerase II",
  "gene_name": "Methylcytosine dioxygenase TET3",
  "gene_symbol": "TET3"
}